{
  "gene": "UniProtKB:P35670",
  "gene_name": "Copper-transporting ATPase 2",
  "term_label": "copper ion binding",
  "term_id": "GO:0005507",
  "gene_symbol": "ATP7B"
}